{
  "gene_symbol": "GBP7",
  "gene": "UniProtKB:Q8N8V2",
  "term_label": "GTPase activity",
  "term_id": "GO:0003924",
  "gene_name": "Guanylate-binding protein 7"
}